{
  "gene_name": "E3 ubiquitin-protein ligase parkin",
  "gene_symbol": "PRKN",
  "term_id": "GO:0000423",
  "gene": "UniProtKB:O60260",
  "term_label": "mitophagy"
}